{
  "gene_name": "Myotonin-protein kinase",
  "gene": "UniProtKB:Q09013",
  "term_label": "regulation of skeletal muscle contraction by calcium ion signaling",
  "gene_symbol": "DMPK",
  "term_id": "GO:0014722"
}